{
  "gene_name": "Lysine--tRNA ligase",
  "gene": "UniProtKB:Q15046",
  "term_label": "lysyl-tRNA aminoacylation",
  "term_id": "GO:0006430",
  "gene_symbol": "KARS1"
}